{
  "term_id": "GO:0005886",
  "term_label": "plasma membrane",
  "gene_symbol": "PACSIN3",
  "gene": "UniProtKB:Q9UKS6",
  "gene_name": "Protein kinase C and casein kinase substrate in neurons protein 3"
}